{
  "term_label": "Unknown biological process",
  "gene": "UniProtKB:Q5VTL8",
  "gene_name": "Pre-mRNA-splicing factor 38B",
  "gene_symbol": "PRPF38B",
  "term_id": "UNKNOWN:0002"
}